{
  "term_id": "GO:0045165",
  "gene_name": "Transcription factor GATA-6",
  "term_label": "cell fate commitment",
  "gene_symbol": "GATA6",
  "gene": "UniProtKB:Q92908"
}